pyrroloquinoline quinone binding [GO:0070968] (molecular function) Sources: GOC:dh Relationships: is a type of carboxylic acid binding [GO:0031406]; is a type of heterocyclic compound binding [GO:1901363] Definition: Binding to pyrroloquinoline quinone, PQQ, the coenzyme or the prosthetic group of certain alcohol dehydrogenases and glucose dehydrogenases. Also known as: PQQ binding